{
  "term_id": "GO:0003924",
  "gene": "UniProtKB:P08240",
  "gene_symbol": "SRPRA",
  "gene_name": "Signal recognition particle receptor subunit alpha",
  "term_label": "GTPase activity"
}